myostimulatory hormone activity [GO:0016084] (molecular function) Relationships: is a type of GO:0005179 Definition: The action characteristic of myostimulatory hormone, a peptide hormone that stimulates muscle contraction. References: PMID:12204246 Sources: GOC:mah